positive regulation of immune system process [GO:0002684] (biological process) Relationships: is a type of regulation of immune system process [GO:0002682]; is a type of positive regulation of biological process [GO:0048518]; positively regulates GO:0002376 Definition: Any process that activates or increases the frequency, rate, or extent of an immune system process. Also known as: up regulation of immune system process, up-regulation of immune system process, upregulation of immune system process, activation of immune system process, stimulation of immune system process Sources: GOC:add Subtypes: GO:0002579, positive regulation of tolerance induction [GO:0002645], positive regulation of leukocyte migration [GO:0002687], positive regulation of leukocyte activation [GO:0002696], positive regulation of immune effector process [GO:0002699], positive regulation of mature B cell apoptotic process [GO:0002907], GO:0033027, positive regulation of neutrophil apoptotic process [GO:0033031], positive regulation of erythrocyte clearance [GO:0034108], positive regulation of hemocyte proliferation [GO:0035208], positive regulation of hemocyte differentiation [GO:0045612], positive regulation of immune response [GO:0050778], GO:0070237, positive regulation of activated T cell autonomous cell death [GO:0070241], positive regulation of hemopoiesis [GO:1903708]